{
  "gene": "UniProtKB:Q9Y2Q0",
  "term_label": "trans-Golgi network",
  "term_id": "GO:0005802",
  "gene_name": "Phospholipid-transporting ATPase IA",
  "gene_symbol": "ATP8A1"
}